translation release factor activity, codon specific [GO:0016149] (MF) Definition: A translation release factor that is specific for one or more particular termination codons; acts at the ribosomal A-site and require polypeptidyl-tRNA at the P-site. Relationships: is a type of translation release factor activity [GO:0003747] Sources: ISBN:0198547684